{
  "gene_symbol": "RAB27B",
  "gene": "UniProtKB:O00194",
  "term_id": "GO:0006887",
  "gene_name": "Ras-related protein Rab-27B",
  "term_label": "exocytosis"
}